{
  "gene_name": "Melanoregulin",
  "gene_symbol": "MREG",
  "term_label": "melanosome transport",
  "gene": "UniProtKB:Q8N565",
  "term_id": "GO:0032402"
}